{
  "gene": "UniProtKB:Q92870",
  "term_id": "GO:0005737",
  "gene_symbol": "APBB2",
  "term_label": "cytoplasm",
  "gene_name": "Amyloid beta precursor protein binding family B member 2"
}